adaptive immune response [GO:0002250] (biological process) Regulation: regulated by regulation of adaptive immune response [GO:0002819]; negatively regulated by GO:0002820; positively regulated by positive regulation of adaptive immune response [GO:0002821] Subtypes: adaptive immune response based on somatic recombination of immune receptors built from leucine-rich repeat domains [GO:0002459], adaptive immune response based on somatic recombination of immune receptors built from immunoglobulin superfamily domains [GO:0002460], adaptive immune memory response [GO:0090716], adaptive immune effector response [GO:0090718], GO:0090720 Definition: An immune response mediated by cells expressing specific receptors for antigens produced through a somatic diversification process, and allowing for an enhanced secondary response to subsequent exposures to the same antigen (immunological memory). Also known as: acquired immune response, immune memory response Relationships: is a type of immune response [GO:0006955] Sources: GOC:add, GO_REF:0000022, ISBN:0781735149